{
  "gene": "UniProtKB:Q15326",
  "term_label": "regulation of transcription elongation by RNA polymerase II",
  "term_id": "GO:0034243",
  "gene_symbol": "ZMYND11",
  "gene_name": "Zinc finger MYND domain-containing protein 11"
}